{
  "gene_symbol": "DMTN",
  "gene": "UniProtKB:Q08495",
  "gene_name": "Dematin",
  "term_label": "actin filament binding",
  "term_id": "GO:0051015"
}